{
  "gene": "UniProtKB:O14810",
  "gene_symbol": "CPLX1",
  "term_id": "GO:0043195",
  "term_label": "terminal bouton",
  "gene_name": "Complexin-1"
}